{
  "gene": "UniProtKB:P00797",
  "gene_name": "Renin",
  "term_label": "aspartic-type endopeptidase activity",
  "gene_symbol": "REN",
  "term_id": "GO:0004190"
}